{
  "term_id": "GO:0005886",
  "term_label": "plasma membrane",
  "gene_name": "Opalin",
  "gene": "UniProtKB:Q96PE5",
  "gene_symbol": "OPALIN"
}